{
  "term_id": "UNKNOWN:0001",
  "gene": "UniProtKB:Q15884",
  "term_label": "Unknown molecular function",
  "gene_name": "Endosomal transmembrane epsin interactor 1",
  "gene_symbol": "ENTREP1"
}